{
  "gene_name": "Protein PBDC1",
  "gene_symbol": "PBDC1",
  "term_label": "'de novo' cotranslational protein folding",
  "term_id": "GO:0051083",
  "gene": "UniProtKB:Q9BVG4"
}